{
  "gene": "UniProtKB:Q8IVL1",
  "term_label": "Unknown molecular function",
  "gene_symbol": "NAV2",
  "gene_name": "Neuron navigator 2",
  "term_id": "UNKNOWN:0001"
}